{
  "gene": "UniProtKB:Q9H6X2",
  "gene_symbol": "ANTXR1",
  "gene_name": "Anthrax toxin receptor 1",
  "term_id": "GO:0004888",
  "term_label": "transmembrane signaling receptor activity"
}